{
  "term_label": "microtubule binding",
  "gene_symbol": "EML6",
  "gene": "UniProtKB:Q6ZMW3",
  "gene_name": "Echinoderm microtubule-associated protein-like 6",
  "term_id": "GO:0008017"
}